{
  "gene_name": "Copine-3",
  "gene": "UniProtKB:O75131",
  "gene_symbol": "CPNE3",
  "term_id": "GO:0071277",
  "term_label": "cellular response to calcium ion"
}